{
  "term_id": "UNKNOWN:0003",
  "gene_name": "Deubiquitinase OTUD6B",
  "gene": "UniProtKB:Q8N6M0",
  "term_label": "Unknown cellular component",
  "gene_symbol": "OTUD6B"
}